negative regulation of protein localization to endoplasmic reticulum [GO:1905551] (biological process) Relationships: is a type of negative regulation of protein localization [GO:1903828]; is a type of regulation of protein localization to endoplasmic reticulum [GO:1905550]; negatively regulates GO:0070972 References: PMID:22768340 Sources: GOC:TermGenie, GO_REF:0000058 Definition: Any process that stops, prevents or reduces the frequency, rate or extent of protein localization to endoplasmic reticulum. Also known as: down regulation of protein localisation in endoplasmic reticulum, down regulation of protein localization in ER, down regulation of protein localization in endoplasmic reticulum, down regulation of protein localization to endoplasmic reticulum, down-regulation of protein localisation in endoplasmic reticulum, down-regulation of protein localization in ER, down-regulation of protein localization in endoplasmic reticulum, down-regulation of protein localization to endoplasmic reticulum, downregulation of protein localisation in endoplasmic reticulum, downregulation of protein localization in ER, downregulation of protein localization in endoplasmic reticulum, downregulation of protein localization to endoplasmic reticulum, negative regulation of protein localisation in endoplasmic reticulum, negative regulation of protein localization in ER, negative regulation of protein localization in endoplasmic reticulum, inhibition of protein localisation in endoplasmic reticulum, inhibition of protein localization in ER, inhibition of protein localization in endoplasmic reticulum, inhibition of protein localization to endoplasmic reticulum